{
  "term_id": "GO:0001968",
  "gene": "UniProtKB:P24592",
  "gene_name": "Insulin-like growth factor-binding protein 6",
  "gene_symbol": "IGFBP6",
  "term_label": "fibronectin binding"
}